{
  "gene": "UniProtKB:P19526",
  "term_label": "Unknown cellular component",
  "term_id": "UNKNOWN:0003",
  "gene_name": "Galactoside alpha-(1,2)-fucosyltransferase 1",
  "gene_symbol": "FUT1"
}